{
  "gene": "UniProtKB:Q9NPB3",
  "term_label": "calcium channel regulator activity",
  "gene_symbol": "CABP2",
  "term_id": "GO:0005246",
  "gene_name": "Calcium-binding protein 2"
}